{
  "gene_name": "Krueppel-like factor 8",
  "term_id": "GO:0006357",
  "term_label": "regulation of transcription by RNA polymerase II",
  "gene": "UniProtKB:O95600",
  "gene_symbol": "KLF8"
}